{
  "gene_name": "5'-nucleotidase domain-containing protein 1",
  "gene": "UniProtKB:Q5TFE4",
  "gene_symbol": "NT5DC1",
  "term_label": "Unknown biological process",
  "term_id": "UNKNOWN:0002"
}